{
  "gene_symbol": "SIK1",
  "term_id": "GO:0005634",
  "gene_name": "Serine_threonine-protein kinase SIK1",
  "gene": "UniProtKB:P57059",
  "term_label": "nucleus"
}